{
  "term_id": "UNKNOWN:0002",
  "gene_name": "Olfactory receptor 4F6",
  "gene_symbol": "OR4F6",
  "term_label": "Unknown biological process",
  "gene": "UniProtKB:Q8NGB9"
}